{
  "gene": "UniProtKB:Q15661",
  "gene_name": "Tryptase alpha_beta-1",
  "gene_symbol": "TPSAB1",
  "term_id": "GO:0006508",
  "term_label": "proteolysis"
}